Golgi to ER transport vesicle membrane [GO:0012508] (CC) Definition: The lipid bilayer surrounding a vesicle transporting substances from the Golgi to the ER. Also known as: Golgi to ER constitutive secretory pathway transport vesicle membrane, Golgi to endoplasmic reticulum transport vesicle membrane, Golgi-ER transport vesicle membrane, Golgi-endoplasmic reticulum transport vesicle membrane Relationships: is a type of GO:0030658; is a type of COPI-coated vesicle membrane [GO:0030663]; is part of GO:0030142 Sources: GOC:ai